tolerance induction in mucosal-associated lymphoid tissue [GO:0002401] (biological process) Sources: GOC:jal, ISBN:0781735149 Relationships: is a type of mucosal tolerance induction [GO:0002427] Subtypes: GO:0002394, B cell tolerance induction in mucosal-associated lymphoid tissue [GO:0002402], T cell tolerance induction in mucosal-associated lymphoid tissue [GO:0002403] Also known as: tolerance induction in MALT Definition: Tolerance induction taking place in the mucosal-associated lymphoid tissue (MALT).